{
  "gene_name": "Granulysin",
  "term_label": "antimicrobial humoral immune response mediated by antimicrobial peptide",
  "gene": "UniProtKB:P22749",
  "term_id": "GO:0061844",
  "gene_symbol": "GNLY"
}